{
  "gene_symbol": "TAF1D",
  "gene_name": "TATA box-binding protein-associated factor RNA polymerase I subunit D",
  "term_id": "UNKNOWN:0001",
  "gene": "UniProtKB:Q9H5J8",
  "term_label": "Unknown molecular function"
}